{
  "gene_symbol": "CLINT1",
  "term_label": "endosome",
  "term_id": "GO:0005768",
  "gene": "UniProtKB:Q14677",
  "gene_name": "Clathrin interactor 1"
}